{
  "term_label": "G-protein beta/gamma-subunit complex binding",
  "gene_name": "Guanine nucleotide-binding protein G(t) subunit alpha-3",
  "gene_symbol": "GNAT3",
  "gene": "UniProtKB:A8MTJ3",
  "term_id": "GO:0031683"
}